acetylacetone-cleaving enzyme activity [GO:0033752] (molecular function) Definition: Catalysis of the reaction: pentane-2,4-dione + O2 = acetate + 2-oxopropanal. Also known as: Dke1, acetylacetone dioxygenase activity, acetylacetone-cleaving enzyme, acetylacetone:oxygen oxidoreductase activity, diketone cleaving dioxygenase activity, diketone cleaving enzyme Relationships: is a type of oxidoreductase activity, acting on single donors with incorporation of molecular oxygen, incorporation of two atoms of oxygen [GO:0016702] Sources: EC:1.13.11.50